positive regulation of protein K63-linked ubiquitination [GO:1902523] (biological process) Definition: Any process that activates or increases the frequency, rate or extent of protein K63-linked ubiquitination. Also known as: positive regulation of protein K63-linked polyubiquitination, up regulation of protein K63-linked polyubiquitination, up regulation of protein K63-linked ubiquitination, up-regulation of protein K63-linked polyubiquitination, up-regulation of protein K63-linked ubiquitination, upregulation of protein K63-linked polyubiquitination, upregulation of protein K63-linked ubiquitination, activation of protein K63-linked polyubiquitination, activation of protein K63-linked ubiquitination Relationships: is_a regulation of protein K63-linked ubiquitination [GO:1900044]; is a type of positive regulation of protein polyubiquitination [GO:1902916]; positively regulates protein K63-linked ubiquitination [GO:0070534] References: PMID:21931591 Sources: GOC:TermGenie Note: An example is BIRC2 (UniProt ID Q13490) in PMID:21931591.